membrane raft polarization [GO:0001766] (biological process) Relationships: is a type of GO:0031580 Also known as: lipid raft polarization, membrane polarization Definition: The clustering and aggregation of a membrane into domains. This serves as a mechanism to compartmentalize cellular activities and to establish cell polarity. Subtypes: plasma membrane raft polarization [GO:0044858] References: PMID:12615889